paramesonephric duct development [GO:0061205] (biological process) Definition: The process whose specific outcome is the progression of the paramesonephric duct over time, from its formation to the mature structure. Mullerian ducts (or paramesonephric ducts) are paired ducts of the embryo that run down the lateral sides of the urogenital ridge and terminate at the mullerian eminence in the primitive urogenital sinus. In the female, they will develop to form the fallopian tubes, uterus, cervix, and the upper portion of the vagina; in the male, they are lost. These ducts are made of tissue of mesodermal origin. Also known as: Mullerian duct development Sources: GOC:dph, GOC:yaf Relationships: is a type of developmental process involved in reproduction [GO:0003006]; is_a GO:0035295